toll-like receptor 4 signaling pathway [GO:0034142] (biological process) Definition: The series of molecular signals initiated by a ligand binding to toll-like receptor 4. Relationships: is a type of GO:0140895 Regulation: regulated by regulation of toll-like receptor 4 signaling pathway [GO:0034143]; negatively regulated by negative regulation of toll-like receptor 4 signaling pathway [GO:0034144]; positively regulated by positive regulation of toll-like receptor 4 signaling pathway [GO:0034145] Subtypes: GO:0035660, GO:0035665, GO:0035667, TRAM-dependent toll-like receptor 4 signaling pathway [GO:0035669] References: PMID:16551253, PMID:17328678 Sources: GOC:add Also known as: TLR4 signaling pathway, toll-like receptor 4 signalling pathway